{
  "gene_name": "V-type proton ATPase 116 kDa subunit a 4",
  "term_label": "proton-transporting ATPase activity, rotational mechanism",
  "gene_symbol": "ATP6V0A4",
  "term_id": "GO:0046961",
  "gene": "UniProtKB:Q9HBG4"
}